{
  "gene": "UniProtKB:P30154",
  "gene_symbol": "PPP2R1B",
  "gene_name": "Serine_threonine-protein phosphatase 2A 65 kDa regulatory subunit A beta isoform",
  "term_label": "cytosol",
  "term_id": "GO:0005829"
}